{
  "term_id": "UNKNOWN:0002",
  "gene_name": "Exostosin-2",
  "gene": "UniProtKB:Q93063",
  "term_label": "Unknown biological process",
  "gene_symbol": "EXT2"
}